{
  "gene": "UniProtKB:Q9NXJ5",
  "term_id": "GO:0030163",
  "gene_name": "Pyroglutamyl-peptidase 1",
  "term_label": "protein catabolic process",
  "gene_symbol": "PGPEP1"
}